{
  "gene_name": "FERM and PDZ domain-containing protein 2",
  "term_label": "1-phosphatidylinositol binding",
  "gene_symbol": "FRMPD2",
  "term_id": "GO:0005545",
  "gene": "UniProtKB:Q68DX3"
}